{
  "gene_symbol": "NXF1",
  "gene_name": "Nuclear RNA export factor 1",
  "gene": "UniProtKB:Q9UBU9",
  "term_label": "nucleus",
  "term_id": "GO:0005634"
}